pre-mRNA 3'-splice site binding [GO:0030628] (molecular function) Definition: Binding to a pre-mRNA 3' splice site sequence. Sources: GOC:jl Also known as: pre-mRNA 3' splice site binding Relationships: is a type of pre-mRNA binding [GO:0036002]